{
  "term_label": "response to bacterium",
  "gene_name": "T cell receptor alpha variable 6",
  "gene_symbol": "TRAV6",
  "gene": "UniProtKB:A0A075B6T7",
  "term_id": "GO:0009617"
}